{
  "gene_symbol": "MGAT4B",
  "gene_name": "Alpha-1,3-mannosyl-glycoprotein 4-beta-N-acetylglucosaminyltransferase B",
  "gene": "UniProtKB:Q9UQ53",
  "term_id": "GO:0005795",
  "term_label": "Golgi stack"
}